{
  "term_id": "GO:0019706",
  "gene": "UniProtKB:P0C7U3",
  "gene_symbol": "ZDHHC11B",
  "gene_name": "Probable palmitoyltransferase ZDHHC11B",
  "term_label": "protein-cysteine S-palmitoyltransferase activity"
}